cellular response to dsDNA [GO:1990786] (biological process) Definition: Any process that results in a change in state or activity of a cell (in terms of movement, secretion, enzyme production, gene expression, etc.) as a result of a double-stranded DNA stimulus. References: PMID:10051633 Relationships: is a type of cellular response to nitrogen compound [GO:1901699]; is a type of response to dsDNA [GO:1990784]